copper ion transport [GO:0006825] (biological process) Relationships: is a type of GO:0000041 Sources: GOC:ai Definition: The directed movement of copper (Cu) ions into, out of or within a cell, or between cells, by means of some agent such as a transporter or pore. Subtypes: copper ion import [GO:0015677], copper ion transmembrane transport [GO:0035434], GO:0097716, copper ion transport across blood-cerebrospinal fluid barrier [GO:0097717]